{
  "gene_name": "Ataxin-8",
  "gene": "UniProtKB:Q156A1",
  "term_id": "UNKNOWN:0001",
  "gene_symbol": "ATXN8",
  "term_label": "Unknown molecular function"
}